phosphonoacetate metabolic process [GO:0019636] (biological process) Definition: The chemical reactions and pathways involving phosphonoacetate, C2H4PO5, a substance composed of an acetate and a phosphonic acid residue. Sources: MetaCyc:P483-PWY Also known as: phosphonoacetate metabolism Relationships: is a type of phosphorus metabolic process [GO:0006793]; is a type of monocarboxylic acid metabolic process [GO:0032787]